negative regulation of caveolin-mediated endocytosis [GO:2001287] (biological process) Also known as: negative regulation of caveolae-dependent endocytosis, negative regulation of caveolae-mediated endocytosis, negative regulation of caveolin-dependent endocytosis Sources: GOC:obol Relationships: is a type of negative regulation of endocytosis [GO:0045806]; is a type of regulation of caveolin-mediated endocytosis [GO:2001286]; negatively regulates GO:0072584 Definition: Any process that stops, prevents or reduces the frequency, rate or extent of caveolin-mediated endocytosis.